{
  "term_label": "actin filament binding",
  "term_id": "GO:0051015",
  "gene_name": "Tubby-related protein 1",
  "gene_symbol": "TULP1",
  "gene": "UniProtKB:O00294"
}